{
  "term_id": "GO:0005096",
  "gene_name": "Ras GTPase-activating-like protein IQGAP2",
  "term_label": "GTPase activator activity",
  "gene_symbol": "IQGAP2",
  "gene": "UniProtKB:Q13576"
}